Y-shaped link assembly [GO:1905350] (biological process) References: PMID:23728985, PMID:24664739, PMID:26595381, PMID:4554367 Sources: GOC:TermGenie, GOC:cilia, GO_REF:0000079 Relationships: is a type of protein-containing complex assembly [GO:0065003] Also known as: Y-shaped link formation, Y-link assembly, Y-link formation, Y-link structure assembly, Y-link structure formation, Y-shaped assemblage assembly, Y-shaped assemblage formation, Y-shaped fiber assembly, Y-shaped fiber formation, Y-shaped fibre assembly, Y-shaped fibre formation, Y-shaped linker assembly, Y-shaped linker formation, membrane-microtubule complex assembly, membrane-microtubule complex formation Definition: The aggregation, arrangement and bonding together of a set of components to form a Y-shaped link. Two distinct protein complexes are known to be involved in proper linker assembly: the MKS complex and the NPHP complex. Improper assembly of Y-shaped links may cause malfunctioning of the transition zone as a molecular gate.